{
  "gene_symbol": "MRAP",
  "gene_name": "Melanocortin-2 receptor accessory protein",
  "term_id": "GO:0031780",
  "gene": "UniProtKB:Q8TCY5",
  "term_label": "corticotropin hormone receptor binding"
}